{
  "gene": "UniProtKB:Q5VYY1",
  "term_id": "UNKNOWN:0001",
  "gene_symbol": "ANKRD22",
  "gene_name": "Ankyrin repeat domain-containing protein 22",
  "term_label": "Unknown molecular function"
}